cardiac muscle hypertrophy [GO:0003300] (biological process) Definition: The enlargement or overgrowth of all or part of the heart muscle due to an increase in size of cardiac muscle cells without cell division. Sources: GOC:mtg_heart Relationships: is_a striated muscle hypertrophy [GO:0014897] Subtypes: physiological cardiac muscle hypertrophy [GO:0003301], cardiac muscle hypertrophy in response to stress [GO:0014898] Regulation: regulated by regulation of cardiac muscle hypertrophy [GO:0010611]; positively regulated by positive regulation of cardiac muscle hypertrophy [GO:0010613]; negatively regulated by negative regulation of cardiac muscle hypertrophy [GO:0010614]